{
  "gene_name": "Tensin-4",
  "gene": "UniProtKB:Q8IZW8",
  "gene_symbol": "TNS4",
  "term_label": "Unknown molecular function",
  "term_id": "UNKNOWN:0001"
}